symbiont-mediated perturbation of host induced systemic resistance [GO:0052159] (biological process) Definition: A process in which a symbiont alters or subverts the induced systemic resistance in the host organism; induced systemic resistance is a response that confers broad spectrum systemic resistance to disease and that does not depend upon salicylic acid signaling. The host is defined as the larger of the organisms involved in a symbiotic interaction. Relationships: is a type of symbiont-mediated perturbation of host immune response [GO:0052553] Also known as: modulation by organism of induced systemic resistance in other organism involved in symbiotic interaction, modulation by symbiont of induced systemic resistance in host, perturbation of host induced systemic resistance Subtypes: symbiont-mediated activation of host induced systemic resistance [GO:0052103] Sources: GOC:mtg_pamgo_17jul06